negative regulation of antigen processing and presentation of lipid antigen via MHC class Ib [GO:0002599] (BP) Definition: Any process that stops, prevents, or reduces the frequency, rate, or extent of antigen processing and presentation of lipid antigen via MHC class Ib. Relationships: is a type of negative regulation of antigen processing and presentation via MHC class Ib [GO:0002593]; is a type of regulation of antigen processing and presentation of lipid antigen via MHC class Ib [GO:0002598]; negatively regulates antigen processing and presentation of lipid antigen via MHC class Ib [GO:0048003] Sources: GOC:add Also known as: down regulation of antigen processing and presentation of lipid antigen via MHC class Ib, down-regulation of antigen processing and presentation of lipid antigen via MHC class Ib, downregulation of antigen processing and presentation of lipid antigen via MHC class Ib, negative regulation of lipid antigen processing and presentation via MHC class Ib, inhibition of antigen processing and presentation of lipid antigen via MHC class Ib